imaginal disc-derived appendage development [GO:0048737] (biological process) Subtypes: GO:0007482 Sources: GOC:jid, GOC:mtg_sensu, GOC:rc Relationships: is a type of appendage development [GO:0048736] Definition: The process whose specific outcome is the progression of an appendage over time, from its formation in the imaginal disc to the mature structure. An appendage is an organ or part that is attached to the trunk of an organism.